{
  "term_id": "GO:0006805",
  "gene": "UniProtKB:Q96SQ9",
  "gene_symbol": "CYP2S1",
  "gene_name": "Cytochrome P450 2S1",
  "term_label": "xenobiotic metabolic process"
}